{
  "gene_symbol": "SNX4",
  "gene_name": "Sorting nexin-4",
  "term_label": "early endosome membrane",
  "term_id": "GO:0031901",
  "gene": "UniProtKB:O95219"
}